eye-antennal disc morphogenesis [GO:0007455] (biological process) Relationships: is a type of imaginal disc morphogenesis [GO:0007560]; is part of GO:0035214 Also known as: eye-antennal disc metamorphosis Sources: GOC:bf, ISBN:0879694238 Definition: The process in which the anatomical structures derived from the eye-antennal disc are generated and organized. This includes the transformation of an eye-antennal imaginal disc from a monolayered epithelium in the larvae of holometabolous insects into recognizable adult structures including the eye, antenna, head capsule and maxillary palps.